{
  "gene": "UniProtKB:A0A5F9ZHS7",
  "gene_symbol": "NFILZ",
  "term_label": "circadian rhythm",
  "gene_name": "NFIL3 like protein",
  "term_id": "GO:0007623"
}